{
  "gene_symbol": "PTEN",
  "gene_name": "Phosphatidylinositol 3,4,5-trisphosphate 3-phosphatase and dual-specificity protein phosphatase PTEN",
  "gene": "UniProtKB:P60484",
  "term_label": "cytosol",
  "term_id": "GO:0005829"
}